{
  "term_label": "nucleoplasm",
  "gene": "UniProtKB:Q6ZSB9",
  "gene_name": "Zinc finger and BTB domain-containing protein 49",
  "gene_symbol": "ZBTB49",
  "term_id": "GO:0005654"
}